{
  "term_label": "metalloendopeptidase inhibitor activity",
  "gene_symbol": "LXN",
  "term_id": "GO:0008191",
  "gene_name": "Latexin",
  "gene": "UniProtKB:Q9BS40"
}